{
  "gene_name": "Keratin, type I cytoskeletal 19",
  "gene_symbol": "KRT19",
  "term_id": "GO:0002009",
  "term_label": "morphogenesis of an epithelium",
  "gene": "UniProtKB:P08727"
}